elaioplast [GO:0009545] (cellular component) Definition: A leucoplast in which oil is stored. Sources: ISBN:0140514031 Relationships: is_a leucoplast [GO:0009516]